{
  "term_label": "visual perception",
  "gene_symbol": "NXNL2",
  "gene": "UniProtKB:Q5VZ03",
  "gene_name": "Nucleoredoxin-like protein 2",
  "term_id": "GO:0007601"
}